{
  "gene": "UniProtKB:Q14344",
  "gene_name": "Guanine nucleotide-binding protein subunit alpha-13",
  "term_id": "GO:0031752",
  "term_label": "D5 dopamine receptor binding",
  "gene_symbol": "GNA13"
}